{
  "term_id": "UNKNOWN:0003",
  "gene_symbol": "LRRC72",
  "gene_name": "Leucine-rich repeat-containing protein 72",
  "gene": "UniProtKB:A6NJI9",
  "term_label": "Unknown cellular component"
}